{
  "term_label": "Unknown biological process",
  "gene_name": "Muscular LMNA-interacting protein",
  "gene": "UniProtKB:Q5VWP3",
  "term_id": "UNKNOWN:0002",
  "gene_symbol": "MLIP"
}